{
  "gene_symbol": "POLD1",
  "gene_name": "DNA polymerase delta catalytic subunit",
  "term_label": "DNA-directed DNA polymerase activity",
  "term_id": "GO:0003887",
  "gene": "UniProtKB:P28340"
}